(R)-sulfopropanediol 2-dehydrogenase activity [GO:0102157] (MF) References: PMID:20150239 Sources: GOC:pz Relationships: is a type of oxidoreductase activity, acting on the CH-OH group of donors, NAD or NADP as acceptor [GO:0016616] Definition: Catalysis of the reaction: (2R)-3-sulfopropanediol(1-) + NAD = 2-oxo-3-hydroxy-propane-1-sulfonate + NADH + H+.